{
  "term_label": "positive regulation of systemic arterial blood pressure",
  "gene_name": "Angiotensin-converting enzyme",
  "gene": "UniProtKB:P12821",
  "term_id": "GO:0003084",
  "gene_symbol": "ACE"
}